symbiont-mediated suppression of host PKR/eIFalpha signaling [GO:0039580] (biological process) Definition: A process in which a symbiont inhibits or disrupts host PKR (Protein Kinase regulated by RNA) signaling. PKR phosphorylates host targets such as the translation initiation factor eIF2alpha that inhibits protein synthesis as an antimicrobial response. Inhibition of host PKR signaling maintains the host ability to translate mRNA. The host is defined as the larger of the organisms involved in a symbiotic interaction. Also known as: suppression by virus of host EIF2AK2 activity, suppression by virus of host PKR activity, suppression by virus of host PKR signaling Relationships: is a type of symbiont-mediated suppression of host signal transduction pathway [GO:0052029]; is a type of symbiont-mediated suppression of host-directed shutoff of host translation [GO:0141154] References: PMID:15207627